{
  "term_label": "sulfate transmembrane transport",
  "gene_symbol": "SLC26A4",
  "gene_name": "Pendrin",
  "gene": "UniProtKB:O43511",
  "term_id": "GO:1902358"
}